keratan-sulfate endo-1,4-beta-galactosidase activity [GO:0033930] (molecular function) Sources: EC:3.2.1.103 Definition: Catalysis of the endohydrolysis of (1->4)-beta-D-galactosidic linkages in keratan sulfate. Also known as: endo-beta-galactosidase activity, keratan sulfate endogalactosidase activity, keratan-sulfate 1,4-beta-D-galactanohydrolase activity, keratanase activity Relationships: is a type of galactosidase activity [GO:0015925]